{
  "gene_name": "DNA damage-binding protein 2",
  "gene": "UniProtKB:Q92466",
  "term_id": "GO:0005634",
  "gene_symbol": "DDB2",
  "term_label": "nucleus"
}